octanol biosynthetic process [GO:0046171] (biological process) Definition: The chemical reactions and pathways resulting in the formation of octanol, the 8-carbon alcohol with the formula C8H17OH. Relationships: is a type of octanol metabolic process [GO:0006070]; is_a primary alcohol biosynthetic process [GO:0034309]; is a type of fatty alcohol biosynthetic process [GO:1903175] Sources: GOC:ai Also known as: octanol anabolism, octanol biosynthesis, octanol formation, octanol synthesis